{
  "gene_name": "SCO-spondin",
  "term_id": "GO:0031012",
  "gene_symbol": "SSPOP",
  "term_label": "extracellular matrix",
  "gene": "UniProtKB:A2VEC9"
}